larval behavior [GO:0030537] (biological process) Definition: Behavior in a larval form of an organism, an immature organism that must undergo metamorphosis to assume adult characteristics. Also known as: larval behaviour Sources: GOC:mah, ISBN:0877797099 Relationships: is a type of behavior [GO:0007610] Subtypes: GO:0008345, larval feeding behavior [GO:0030536], larval foraging behavior [GO:0035177] Note: See also the biological process term 'behavior ; GO:0007610'.